RNA-(apurinic or apyrimidinic site) endonuclease activity [GO:0052719] (molecular function) Relationships: is a type of RNA endonuclease activity producing 5'-phosphomonoesters, hydrolytic mechanism [GO:0016891] References: PMID:19401441 Definition: Catalysis of the hydrolysis of ester linkages immediately 5' to an apurinic/apyrimidinic (AP; also called abasic) site within a ribonucleic acid molecule by creating internal breaks, generating a single-strand break with 5'-ribose phosphate and 3'-hydroxyl ends. Also known as: AP endoribonuclease activity, abasic endoribonuclease activity, apurinic endoribonuclease activity, apyrimidinic endoribonuclease activity